{
  "gene_name": "Putative uncharacterized protein FLJ45256",
  "gene": "UniProtKB:Q6ZSR6",
  "term_id": "UNKNOWN:0001",
  "gene_symbol": "Q6ZSR6",
  "term_label": "Unknown molecular function"
}